{
  "term_label": "regulation of cell population proliferation",
  "gene": "UniProtKB:Q92481",
  "gene_symbol": "TFAP2B",
  "gene_name": "Transcription factor AP-2-beta",
  "term_id": "GO:0042127"
}